{
  "gene": "UniProtKB:Q9UPC5",
  "gene_symbol": "GPR34",
  "term_label": "G protein-coupled receptor signaling pathway",
  "gene_name": "Probable G-protein coupled receptor 34",
  "term_id": "GO:0007186"
}